mediator complex [GO:0016592] (cellular component) Definition: A protein complex that interacts with the carboxy-terminal domain of the largest subunit of RNA polymerase II and plays an active role in transducing the signal from a transcription factor to the transcriptional machinery. The mediator complex is required for activation of transcription of most protein-coding genes, but can also act as a transcriptional corepressor. The Saccharomyces complex contains several identifiable subcomplexes: a head domain comprising Srb2, -4, and -5, Med6, -8, and -11, and Rox3 proteins; a middle domain comprising Med1, -4, and -7, Nut1 and -2, Cse2, Rgr1, Soh1, and Srb7 proteins; a tail consisting of Gal11p, Med2p, Pgd1p, and Sin4p; and a regulatory subcomplex comprising Ssn2, -3, and -8, and Srb8 proteins. Metazoan mediator complexes have similar modular structures and include homologs of yeast Srb and Med proteins. References: PMID:11454195, PMID:16168358, PMID:17870225 Also known as: L mediator complex, Srb-mediator complex, TRAP complex, CDK8-containing TRAP/mediator complex Relationships: is a type of nuclear protein-containing complex [GO:0140513]; has part core mediator complex [GO:0070847]